{
  "term_label": "ruffle membrane",
  "gene_name": "Allograft inflammatory factor 1-like",
  "term_id": "GO:0032587",
  "gene_symbol": "AIF1L",
  "gene": "UniProtKB:Q9BQI0"
}